{
  "gene": "UniProtKB:Q06520",
  "gene_name": "Sulfotransferase 2A1",
  "term_label": "cytoplasm",
  "term_id": "GO:0005737",
  "gene_symbol": "SULT2A1"
}